{
  "gene_name": "Ribosomal biogenesis protein LAS1L",
  "gene_symbol": "LAS1L",
  "term_id": "GO:0005634",
  "term_label": "nucleus",
  "gene": "UniProtKB:Q9Y4W2"
}